mandelate 4-monooxygenase activity [GO:0050481] (MF) Definition: Catalysis of the reaction: (S)-mandelate + 5,6,7,8-tetrahydrobiopterin + O2 = (S)-4-hydroxymandelate + 7,8-dihydrobiopterin + H2O. (S)-2-hydroxy-2-phenylacetate is also known as S-mandelate. Sources: EC:1.14.16.6, RHEA:21716 Also known as: L-mandelate 4-hydroxylase activity, (S)-2-hydroxy-2-phenylacetate,tetrahydrobiopterin:oxygen oxidoreductase (4-hydroxylating), mandelic acid 4-hydroxylase activity Relationships: is a type of oxidoreductase activity, acting on paired donors, with incorporation or reduction of molecular oxygen, reduced pteridine as one donor, and incorporation of one atom of oxygen [GO:0016714]